{
  "gene": "UniProtKB:Q16134",
  "term_label": "electron transport chain",
  "term_id": "GO:0022900",
  "gene_symbol": "ETFDH",
  "gene_name": "Electron transfer flavoprotein-ubiquinone oxidoreductase, mitochondrial"
}